{
  "term_label": "nuclear pore",
  "gene_symbol": "NUP50",
  "gene_name": "Nuclear pore complex protein Nup50",
  "gene": "UniProtKB:Q9UKX7",
  "term_id": "GO:0005643"
}